meiotic recombination initiation complex [GO:0035808] (cellular component) References: PMID:12897161, PMID:20364342, PMID:21429938 Sources: GOC:vw Definition: A protein complex that initiates the formation of double-strand breaks (DSBs) required for meiotic recombination. Consists of a protein that catalyses formation of the double-strand breaks (Spo11 in S. cerevisiae and Rec12 in S. pombe), and a number of accessory proteins. Relationships: is a type of nuclear protein-containing complex [GO:0140513]; is part of condensed nuclear chromosome [GO:0000794]